{
  "gene_symbol": "DLX6",
  "term_label": "nucleus",
  "gene": "UniProtKB:P56179",
  "term_id": "GO:0005634",
  "gene_name": "Homeobox protein DLX-6"
}